{
  "gene": "UniProtKB:P61586",
  "term_id": "GO:0019901",
  "term_label": "protein kinase binding",
  "gene_name": "Transforming protein RhoA",
  "gene_symbol": "RHOA"
}